{
  "term_id": "GO:0034338",
  "term_label": "short-chain carboxylesterase activity",
  "gene": "UniProtKB:Q6UXT9",
  "gene_symbol": "ABHD15",
  "gene_name": "Protein ABHD15"
}